{
  "gene": "UniProtKB:Q9Y2P0",
  "term_label": "RNA polymerase II cis-regulatory region sequence-specific DNA binding",
  "gene_name": "Zinc finger protein 835",
  "term_id": "GO:0000978",
  "gene_symbol": "ZNF835"
}